enteric nervous system development [GO:0048484] (biological process) Sources: FMA:66070, GOC:jid, GOC:sr Relationships: is a type of system development [GO:0048731]; is part of autonomic nervous system development [GO:0048483] Definition: The process whose specific outcome is the progression of the enteric nervous system over time, from its formation to the mature structure. The enteric nervous system is composed of two ganglionated neural plexuses in the gut wall which form one of the three major divisions of the autonomic nervous system. The enteric nervous system innervates the gastrointestinal tract, the pancreas, and the gallbladder. It contains sensory neurons, interneurons, and motor neurons. Thus the circuitry can autonomously sense the tension and the chemical environment in the gut and regulate blood vessel tone, motility, secretions, and fluid transport. The system is itself governed by the central nervous system and receives both parasympathetic and sympathetic innervation.